{
  "gene_symbol": "PLCB1",
  "term_id": "GO:0005737",
  "gene": "UniProtKB:Q9NQ66",
  "gene_name": "1-phosphatidylinositol 4,5-bisphosphate phosphodiesterase beta-1",
  "term_label": "cytoplasm"
}